mitochondrial inner membrane [GO:0005743] (cellular component) Sources: GOC:ai Also known as: inner mitochondrial membrane, inner mitochondrion membrane, mitochondrion inner membrane Relationships: is a type of organelle inner membrane [GO:0019866]; is a type of mitochondrial membrane [GO:0031966] Definition: The inner, i.e. lumen-facing, lipid bilayer of the mitochondrial envelope. It is highly folded to form cristae.